{
  "term_label": "regulation of transcription by RNA polymerase II",
  "gene_symbol": "ZNF790",
  "gene_name": "Zinc finger protein 790",
  "term_id": "GO:0006357",
  "gene": "UniProtKB:Q6PG37"
}